{
  "term_label": "Golgi apparatus",
  "term_id": "GO:0005794",
  "gene_symbol": "PLOD2",
  "gene": "UniProtKB:O00469",
  "gene_name": "Procollagen-lysine,2-oxoglutarate 5-dioxygenase 2"
}